{
  "gene_name": "CUB and sushi domain-containing protein 1",
  "gene_symbol": "CSMD1",
  "gene": "UniProtKB:Q96PZ7",
  "term_label": "Unknown biological process",
  "term_id": "UNKNOWN:0002"
}